{
  "gene_symbol": "MFSD14CP",
  "gene_name": "Major facilitator superfamily domain-containing 14C pseudogene",
  "term_label": "Unknown biological process",
  "gene": "UniProtKB:Q5VZR4",
  "term_id": "UNKNOWN:0002"
}